regulation of integrin activation [GO:0033623] (biological process) Also known as: regulation of integrin complex activation Definition: Any process that modulates the frequency, rate, or extent of integrin activation. Relationships: is a type of regulation of protein-containing complex assembly [GO:0043254]; regulates integrin activation [GO:0033622] Sources: GOC:add Subtypes: negative regulation of integrin activation [GO:0033624], positive regulation of integrin activation [GO:0033625]